polyadenylation of viral mRNA by polymerase stuttering [GO:0039698] (biological process) Sources: VZ:1916 Relationships: is a type of GO:0016032 Definition: Polyadenylation of viral mRNA through a polymerase stuttering mechanism. The stop signal present at the end of each gene comprises a stretch of uridine on which the viral polymerase acquires a stuttering behavior: after each adenine inserted, the polymerase moves back one nucleotide along with the mRNA. It resumes transcription adding a new adenine, then again moves back, thereby producing a polyA tail. Also known as: polyA stuttering